{
  "gene_name": "tRNA pseudouridine synthase-like 1",
  "gene_symbol": "PUSL1",
  "term_id": "UNKNOWN:0003",
  "gene": "UniProtKB:Q8N0Z8",
  "term_label": "Unknown cellular component"
}